{
  "gene": "UniProtKB:Q86WR6",
  "gene_name": "CHD1 helical C-terminal domain containing protein 1",
  "term_id": "UNKNOWN:0003",
  "term_label": "Unknown cellular component",
  "gene_symbol": "CHCT1"
}